{
  "gene_symbol": "TRIM17",
  "term_id": "GO:0061630",
  "gene": "UniProtKB:Q9Y577",
  "gene_name": "E3 ubiquitin-protein ligase TRIM17",
  "term_label": "ubiquitin protein ligase activity"
}